{
  "gene_name": "C-C chemokine receptor type 1",
  "gene": "UniProtKB:P32246",
  "gene_symbol": "CCR1",
  "term_label": "chemokine (C-C motif) ligand 7 binding",
  "term_id": "GO:0035717"
}